{
  "gene": "UniProtKB:P55055",
  "gene_symbol": "NR1H2",
  "term_id": "GO:0030154",
  "gene_name": "Oxysterols receptor LXR-beta",
  "term_label": "cell differentiation"
}